 [go#gocheck:obsoletion:candidate] Note: Terms planned for obsoletion